{
  "term_id": "UNKNOWN:0003",
  "gene": "UniProtKB:O00587",
  "gene_name": "Beta-1,3-N-acetylglucosaminyltransferase manic fringe",
  "term_label": "Unknown cellular component",
  "gene_symbol": "MFNG"
}